{
  "gene_symbol": "ZFP57",
  "term_id": "GO:0005634",
  "gene_name": "Zinc finger protein 57 homolog",
  "term_label": "nucleus",
  "gene": "UniProtKB:Q9NU63"
}